{
  "term_label": "Unknown molecular function",
  "term_id": "UNKNOWN:0001",
  "gene_symbol": "CECR2",
  "gene_name": "Chromatin remodeling regulator CECR2",
  "gene": "UniProtKB:Q9BXF3"
}